positive regulation of cardiac muscle hypertrophy [GO:0010613] (biological process) Relationships: is a type of regulation of cardiac muscle hypertrophy [GO:0010611]; is a type of GO:0014742; positively regulates GO:0003300 Definition: Any process that increases the rate, frequency or extent of the enlargement or overgrowth of all or part of the heart due to an increase in size (not length) of individual cardiac muscle fibers, without cell division. Subtypes: GO:0061051, positive regulation of cardiac muscle hypertrophy in response to stress [GO:1903244] Sources: GOC:BHF, GOC:dph, GOC:tb